aliphatic (R)-hydroxynitrile lyase activity [GO:0052919] (MF) Definition: Catalysis of the reaction: an aliphatic (R)-hydroxynitrile = an aliphatic aldehyde or ketone + hydrogen cyanide. Sources: EC:4.1.2.46 Also known as: (R)-HNL activity, (R)-hydroxynitrile lyase activity, (R)-oxynitrilase activity Relationships: is a type of GO:0016832